{
  "gene_symbol": "ADGRL2",
  "term_label": "G protein-coupled receptor activity",
  "gene": "UniProtKB:O95490",
  "gene_name": "Adhesion G protein-coupled receptor L2",
  "term_id": "GO:0004930"
}